{
  "term_label": "DNA-binding transcription factor activity",
  "gene": "UniProtKB:Q96AP4",
  "term_id": "GO:0003700",
  "gene_name": "Zinc finger-containing ubiquitin peptidase 1",
  "gene_symbol": "ZUP1"
}